teichoic acid D-alanylation [GO:0070400] (biological process) Subtypes: GO:0036358 References: PMID:14665680, PMID:16020688 Sources: GOC:add Relationships: is a type of teichoic acid biosynthetic process [GO:0019350] Definition: The formation of a D-alanyl ester of teichoic acid. Alanylation of teichoic acids modulates the properties of the bacterial cell wall and modulates the inflammatory properties of the teichoic acid. Also known as: teichoic acid alanylation